{
  "gene": "UniProtKB:Q99714",
  "gene_symbol": "HSD17B10",
  "term_label": "estrogen metabolic process",
  "term_id": "GO:0008210",
  "gene_name": "3-hydroxyacyl-CoA dehydrogenase type-2"
}